{
  "term_label": "GTPase activity",
  "gene": "UniProtKB:Q96F15",
  "term_id": "GO:0003924",
  "gene_symbol": "GIMAP5",
  "gene_name": "GTPase IMAP family member 5"
}